{
  "term_id": "GO:0005814",
  "gene": "UniProtKB:Q9UPV0",
  "gene_symbol": "CEP164",
  "gene_name": "Centrosomal protein of 164 kDa",
  "term_label": "centriole"
}